ferricrocin biosynthetic process [GO:0031171] (biological process) Definition: The chemical reactions and pathways resulting in the formation of ferricrocin, a cyclic hexapeptide siderophore with the structure Gly-Ser-Gly-(N5-acetyl-N5-hydroxyornithine)3. Also known as: ferricrocin anabolism, ferricrocin biosynthesis, ferricrocin formation, ferricrocin synthesis, ferricrocin biosynthetic process, peptide formation, ferricrocin biosynthetic process, peptide modification Relationships: is a type of ferrichrome biosynthetic process [GO:0031169] References: PMID:12828635 Sources: GOC:mah Regulation: regulated by GO:1900678; negatively regulated by negative regulation of ferricrocin biosynthetic process [GO:1900679]; positively regulated by positive regulation of ferricrocin biosynthetic process [GO:1900680]